{
  "term_id": "GO:0030971",
  "gene_symbol": "ANGPT1",
  "gene_name": "Angiopoietin-1",
  "term_label": "receptor tyrosine kinase binding",
  "gene": "UniProtKB:Q15389"
}